ureter development [GO:0072189] (biological process) Relationships: is a type of tube development [GO:0035295]; is a type of animal organ development [GO:0048513]; is part of renal system development [GO:0072001] Sources: GOC:mtg_kidney_jan10 Definition: The process whose specific outcome is the progression of the ureter over time, from its formation to the mature structure. The ureter is a muscular tube that transports urine from the kidney to the urinary bladder or from the Malpighian tubule to the hindgut.